{
  "gene_name": "Zinc finger protein 443",
  "term_label": "RNA polymerase II transcription regulatory region sequence-specific DNA binding",
  "term_id": "GO:0000977",
  "gene_symbol": "ZNF443",
  "gene": "UniProtKB:Q9Y2A4"
}